{
  "term_id": "GO:0043123",
  "term_label": "positive regulation of canonical NF-kappaB signal transduction",
  "gene": "UniProtKB:P01374",
  "gene_symbol": "LTA",
  "gene_name": "Lymphotoxin-alpha"
}